{
  "gene_name": "Solute carrier family 35 member F5",
  "term_id": "UNKNOWN:0001",
  "term_label": "Unknown molecular function",
  "gene_symbol": "SLC35F5",
  "gene": "UniProtKB:Q8WV83"
}